{
  "gene_name": "NFX1-type zinc finger-containing protein 1",
  "term_label": "RNA binding",
  "term_id": "GO:0003723",
  "gene_symbol": "ZNFX1",
  "gene": "UniProtKB:Q9P2E3"
}